{
  "gene_symbol": "NDUFS5",
  "term_label": "respiratory chain complex I",
  "gene_name": "NADH dehydrogenase [ubiquinone] iron-sulfur protein 5",
  "term_id": "GO:0045271",
  "gene": "UniProtKB:O43920"
}